{
  "gene_symbol": "NKD1",
  "term_label": "negative regulation of Wnt signaling pathway",
  "gene_name": "Protein naked cuticle homolog 1",
  "term_id": "GO:0030178",
  "gene": "UniProtKB:Q969G9"
}